{
  "gene_name": "XK-related protein 4",
  "gene_symbol": "XKR4",
  "term_id": "GO:0070782",
  "gene": "UniProtKB:Q5GH76",
  "term_label": "phosphatidylserine exposure on apoptotic cell surface"
}